{
  "term_label": "Unknown biological process",
  "gene_name": "POTE ankyrin domain family member D",
  "gene_symbol": "POTED",
  "term_id": "UNKNOWN:0002",
  "gene": "UniProtKB:Q86YR6"
}